astrocyte activation [GO:0048143] (biological process) Relationships: is a type of glial cell activation [GO:0061900]; is part of astrocyte development [GO:0014002] References: PMID:10526094, PMID:10695728, PMID:12529254, PMID:12580336, PMID:9585813 Sources: GOC:mgi_curators Definition: A change in morphology and behavior of an astrocyte resulting from exposure to a cytokine, chemokine, cellular ligand, or soluble factor. Subtypes: astrocyte activation involved in immune response [GO:0002265] Regulation: RO_0002211 by regulation of astrocyte activation [GO:0061888]; negatively regulated by negative regulation of astrocyte activation [GO:0061889]; positively regulated by positive regulation of astrocyte activation [GO:0061890]